bone cell development [GO:0098751] (biological process) Relationships: is a type of cell development [GO:0048468]; BFO_0000050 bone development [GO:0060348] Note: Not to be used for manual annotation. Please choose a more specific cell development term or if not possible, bone or bone tissue development. Sources: GOC:dos Subtypes: osteoclast development [GO:0036035] Definition: The process whose specific outcome is the progression of a bone cell over time, from initial commitment of the cell to a specific fate, to the fully functional differentiated cell.